{
  "term_id": "GO:0035725",
  "gene_name": "Sodium channel protein type 9 subunit alpha",
  "term_label": "sodium ion transmembrane transport",
  "gene_symbol": "SCN9A",
  "gene": "UniProtKB:Q15858"
}